{
  "gene": "UniProtKB:Q9BY08",
  "term_id": "GO:0005783",
  "gene_name": "Emopamil-binding protein-like",
  "gene_symbol": "EBPL",
  "term_label": "endoplasmic reticulum"
}